ecgonine methyl ester biosynthetic process [GO:1901869] (biological process) Relationships: is_a tropane alkaloid biosynthetic process [GO:0009710] Also known as: ecgonine methyl ester anabolism, ecgonine methyl ester biosynthesis, ecgonine methyl ester formation, ecgonine methyl ester synthesis Definition: The chemical reactions and pathways resulting in the formation of ecgonine methyl ester. References: PMID:22665766 Sources: GOC:TermGenie